Pup transferase activity [GO:0072496] (molecular function) Definition: Catalysis of the transfer of Pup from one protein to another via the reaction X-Pup + Y = Y-Pup + X, where both X-Pup and Y-Pup are covalent linkages. Sources: GOC:sp Also known as: Pup conjugating enzyme activity Relationships: is a type of ubiquitin-like protein transferase activity [GO:0019787] Subtypes: Pup conjugating enzyme activity [GO:0061655], Pup ligase activity [GO:0061664]